tRNA (guanine(37)-N1)-methyltransferase activity [GO:0052906] (molecular function) Relationships: is a type of tRNA (guanine) methyltransferase activity [GO:0016423] Sources: EC:2.1.1.228 Also known as: tRNA (guanine(37)-N(1))-methyltransferase activity, tRNA (guanosine(37)-N(1))-methyltransferase activity, tRNA (guanosine(37)-N1-)-methyltransferase activity, tRNA (m(1)G(37)) methyltransferase activity, tRNA-(N(1)G37) methyltransferase activity, transfer RNA (m(1)G(37)) methyltransferase activity Definition: Catalysis of the reaction: S-adenosyl-L-methionine + guanine(37) in tRNA = N(1)-methylguanine(37) in tRNA + S-adenosyl-L-homocysteine.